{
  "term_id": "GO:0008286",
  "gene_symbol": "IRS4",
  "gene": "UniProtKB:O14654",
  "term_label": "insulin receptor signaling pathway",
  "gene_name": "Insulin receptor substrate 4"
}